{
  "term_id": "GO:0016081",
  "gene": "UniProtKB:Q9UPW8",
  "gene_name": "Protein unc-13 homolog A",
  "gene_symbol": "UNC13A",
  "term_label": "synaptic vesicle docking"
}